{
  "gene_name": "Myozenin-3",
  "gene_symbol": "MYOZ3",
  "term_label": "actin cytoskeleton",
  "term_id": "GO:0015629",
  "gene": "UniProtKB:Q8TDC0"
}